symbiont-mediated arrest of host cell cycle during G2/M transition [GO:0039592] (biological process) Definition: A process in which a symbiont interferes with the progression of the host mitotic cell cycle from G2 phase to M phase, leading to arrest in G2 phase. The arrest in G2/M allows some viruses to replicate their genome before cells enter mitosis. Alternatively, it can inhibit the antiviral immune response by preventing the clonal expansion of infected lymphocytes. Also known as: host G2/M cell cycle arrest by virus, perturbation by virus of G2/M transition of host mitotic cell cycle, suppression by virus of G2/M transition of host mitotic cell cycle Relationships: is a type of symbiont-mediated perturbation of host cell cycle progression [GO:0044071] References: PMID:10946289, PMID:12208959, PMID:9882364 Sources: VZ:876